{
  "term_label": "cytoplasm",
  "gene": "UniProtKB:P30281",
  "term_id": "GO:0005737",
  "gene_symbol": "CCND3",
  "gene_name": "G1_S-specific cyclin-D3"
}